ADP reductase activity [GO:0051061] (molecular function) Also known as: ADP reduction Relationships: is a type of ribonucleoside-diphosphate reductase activity, thioredoxin disulfide as acceptor [GO:0004748] Sources: MetaCyc:ADPREDUCT-RXN Definition: Catalysis of the reaction: dADP + thioredoxin disulfide + H2O = ADP + thioredoxin.